{
  "gene": "UniProtKB:P21980",
  "term_label": "regulation of apoptotic cell clearance",
  "gene_symbol": "TGM2",
  "gene_name": "Protein-glutamine gamma-glutamyltransferase 2",
  "term_id": "GO:2000425"
}